{
  "gene_symbol": "ITSN2",
  "gene_name": "Intersectin-2",
  "gene": "UniProtKB:Q9NZM3",
  "term_label": "plasma membrane",
  "term_id": "GO:0005886"
}